{
  "gene_name": "AT-rich interactive domain-containing protein 1A",
  "gene_symbol": "ARID1A",
  "term_id": "GO:0016514",
  "term_label": "SWI/SNF complex",
  "gene": "UniProtKB:O14497"
}